{
  "term_label": "microfilament motor activity",
  "term_id": "GO:0000146",
  "gene_symbol": "MYO7A",
  "gene": "UniProtKB:Q13402",
  "gene_name": "Unconventional myosin-VIIa"
}